mitochondrial creatine kinase complex [GO:0002187] (cellular component) Relationships: is a type of creatine kinase complex [GO:0002185]; is a type of mitochondrial protein-containing complex [GO:0098798] Definition: An octomeric protein complex having creatine kinase activity. References: PMID:16236486